{
  "gene_name": "Vascular endothelial growth factor D",
  "gene": "UniProtKB:O43915",
  "term_label": "induction of positive chemotaxis",
  "term_id": "GO:0050930",
  "gene_symbol": "VEGFD"
}